{
  "term_id": "UNKNOWN:0002",
  "gene_name": "FYVE, RhoGEF and PH domain-containing protein 5",
  "term_label": "Unknown biological process",
  "gene": "UniProtKB:Q6ZNL6",
  "gene_symbol": "FGD5"
}